{
  "term_label": "Unknown molecular function",
  "gene_name": "Small integral membrane protein 28",
  "gene": "UniProtKB:A0A1B0GU29",
  "term_id": "UNKNOWN:0001",
  "gene_symbol": "SMIM28"
}